{
  "gene": "UniProtKB:Q86WR7",
  "gene_symbol": "PROSER2",
  "gene_name": "Proline and serine-rich protein 2",
  "term_label": "Unknown molecular function",
  "term_id": "UNKNOWN:0001"
}